{
  "term_label": "apical plasma membrane",
  "gene": "UniProtKB:Q9BYG5",
  "gene_name": "Partitioning defective 6 homolog beta",
  "gene_symbol": "PARD6B",
  "term_id": "GO:0016324"
}